{
  "term_id": "GO:0002502",
  "gene_name": "Tapasin-related protein",
  "gene": "UniProtKB:Q9BX59",
  "gene_symbol": "TAPBPL",
  "term_label": "peptide antigen assembly with MHC class I protein complex"
}